host cell mitochondrion [GO:0033650] (cellular component) Sources: GOC:pamgo_curators Relationships: is a type of host intracellular membrane-bounded organelle [GO:0033648]; is a type of host cell cytoplasm part [GO:0033655] Also known as: host mitochondria Definition: A semiautonomous, self replicating organelle as found in host cells that occurs in varying numbers, shapes, and sizes in the cell cytoplasm. The host is defined as the larger of the organisms involved in a symbiotic interaction.